{
  "gene": "UniProtKB:Q8NBN7",
  "gene_symbol": "RDH13",
  "gene_name": "Retinol dehydrogenase 13",
  "term_id": "GO:0052650",
  "term_label": "all-trans-retinol dehydrogenase (NADP+) activity"
}